{
  "gene_name": "Inhibitor of nuclear factor kappa-B kinase subunit alpha",
  "gene": "UniProtKB:O15111",
  "gene_symbol": "CHUK",
  "term_label": "protein serine/threonine kinase activity",
  "term_id": "GO:0004674"
}